I(KACh) inward rectifier potassium channel complex [GO:1990566] (cellular component) Definition: An inward rectifier potassium channel complex expressed in cardiac muscle, specifically the sinoatrial node and atria, where it controls the heart rate, via regulation by G protein-coupled receptor signaling. In mammals it is composed of GIRK1 (or Kir3.1) and GIRK4 (or Kir3.4) subunits. References: PMID:9765280 Sources: GOC:ame Also known as: GIRK1-GIRK4 G protein-coupled atrial inward rectifier potassium channel complex, Kir3.1-Kir3.4 G protein-coupled atrial inward rectifier potassium channel complex, muscarinic potassium channel complex Note: Examples of this are KCNJ3 and KCNJ5 in human (Uniprot symbols P48549 and P48544) in PMID:9765280 inferred from orthology sequence evidence. Relationships: is a type of inward rectifier potassium channel complex [GO:1902937]